{
  "term_id": "GO:0005886",
  "term_label": "plasma membrane",
  "gene_symbol": "TPRA1",
  "gene_name": "Transmembrane protein adipocyte-associated 1",
  "gene": "UniProtKB:Q86W33"
}